sequestering of nodal from receptor via nodal binding [GO:0038101] (biological process) Relationships: is a type of GO:0035581; BFO_0000050 negative regulation of nodal signaling pathway [GO:1900108]; has part nodal binding [GO:0038100] Also known as: extracellular regulation of nodal, nodal antagonist activity, binding to and sequestering nodal References: PMID:14570583, PMID:15062104 Sources: GOC:signaling Definition: Binding to a nodal protein in the extracellular region, and inhibiting nodal signaling by preventing nodal from binding to its cell surface receptor.